{
  "gene": "UniProtKB:Q8NB90",
  "term_id": "GO:0042273",
  "term_label": "ribosomal large subunit biogenesis",
  "gene_name": "ATPase family gene 2 protein homolog A",
  "gene_symbol": "AFG2A"
}